{
  "term_label": "phospholipid metabolic process",
  "gene": "UniProtKB:Q9NZC3",
  "gene_symbol": "GDE1",
  "gene_name": "Glycerophosphodiester phosphodiesterase 1",
  "term_id": "GO:0006644"
}